{
  "term_id": "GO:0030915",
  "gene": "UniProtKB:Q8IY18",
  "term_label": "Smc5-Smc6 complex",
  "gene_symbol": "SMC5",
  "gene_name": "Structural maintenance of chromosomes protein 5"
}